negative regulation of serine-type endopeptidase activity [GO:1900004] (biological process) Sources: GOC:TermGenie Relationships: is a type of GO:0010951; is a type of regulation of serine-type endopeptidase activity [GO:1900003]; is a type of negative regulation of serine-type peptidase activity [GO:1902572]; negatively regulates GO:0004252 Also known as: down regulation of blood coagulation factor activity, down regulation of serine-type endopeptidase activity, negative regulation of blood coagulation factor activity Definition: Any process that stops, prevents or reduces the frequency, rate or extent of serine-type endopeptidase activity.